{
  "term_label": "Unknown cellular component",
  "gene_symbol": "FUT9",
  "gene_name": "4-galactosyl-N-acetylglucosaminide 3-alpha-L-fucosyltransferase 9",
  "term_id": "UNKNOWN:0003",
  "gene": "UniProtKB:Q9Y231"
}